{
  "term_label": "Unknown cellular component",
  "term_id": "UNKNOWN:0003",
  "gene_symbol": "CRYBG3",
  "gene_name": "Very large A-kinase anchor protein",
  "gene": "UniProtKB:Q68DQ2"
}